{
  "gene_symbol": "ZFP57",
  "term_id": "GO:0006357",
  "gene_name": "Zinc finger protein 57 homolog",
  "gene": "UniProtKB:Q9NU63",
  "term_label": "regulation of transcription by RNA polymerase II"
}